{
  "term_id": "GO:0005634",
  "gene_symbol": "ZNF69",
  "gene_name": "Zinc finger protein 69",
  "gene": "UniProtKB:Q9UC07",
  "term_label": "nucleus"
}